cytoplasmic vesicle membrane [GO:0030659] (cellular component) Definition: The lipid bilayer surrounding a cytoplasmic vesicle. Relationships: is a type of GO:0012506; BFO_0000050 cytoplasmic vesicle [GO:0031410] Subtypes: inner acrosomal membrane [GO:0002079], outer acrosomal membrane [GO:0002081], endosome membrane [GO:0010008], transport vesicle membrane [GO:0030658], GO:0030660, chitosome membrane [GO:0030661], coated vesicle membrane [GO:0030662], GO:0030666, secretory granule membrane [GO:0030667], contractile vacuolar membrane [GO:0031164], aleurone grain membrane [GO:0032578], Cvt vesicle membrane [GO:0033110], GO:0033118, gut granule membrane [GO:0044841], organellar chromatophore membrane [GO:0070112], pigment granule membrane [GO:0090741], multivesicular body, internal vesicle membrane [GO:0097488], GO:0106175, GO:0120202 Sources: GOC:mah